{
  "gene_symbol": "OR5D18",
  "gene": "UniProtKB:Q8NGL1",
  "gene_name": "Olfactory receptor 5D18",
  "term_id": "GO:0004984",
  "term_label": "olfactory receptor activity"
}